{
  "gene": "UniProtKB:Q9UGL1",
  "term_id": "GO:0005634",
  "gene_name": "Lysine-specific demethylase 5B",
  "gene_symbol": "KDM5B",
  "term_label": "nucleus"
}